{
  "term_label": "Unknown molecular function",
  "gene_name": "von Hippel-Lindau-like protein",
  "gene_symbol": "VHLL",
  "term_id": "UNKNOWN:0001",
  "gene": "UniProtKB:Q6RSH7"
}